{
  "gene_name": "B-cell CLL_lymphoma 6 member B protein",
  "term_id": "GO:0042092",
  "term_label": "type 2 immune response",
  "gene_symbol": "BCL6B",
  "gene": "UniProtKB:Q8N143"
}